{
  "gene_name": "Prolactin receptor",
  "term_label": "cytokine-mediated signaling pathway",
  "gene_symbol": "PRLR",
  "term_id": "GO:0019221",
  "gene": "UniProtKB:P16471"
}